deacetylcephalosporin-C acetyltransferase activity [GO:0033813] (molecular function) Sources: EC:2.3.1.175, RHEA:23860 Also known as: CPC acetylhydrolase activity, DAC acetyltransferase activity, DAC-AT, acetyl coenzyme A:DAC acetyltransferase activity, acetyl-CoA:DAC O-acetyltransferase activity, acetyl-CoA:DAC acetyltransferase activity, acetyl-CoA:deacetylcephalosporin-C O-acetyltransferase activity, acetyl-CoA:deacetylcephalosporin-C acetyltransferase activity, cefG, deacetylcephalosporin C acetyltransferase activity Definition: Catalysis of the reaction: acetyl-CoA + deacetylcephalosporin C = cephalosporin C + CoA. Relationships: is a type of GO:0016408